{
  "gene": "UniProtKB:Q96AP0",
  "gene_name": "Adrenocortical dysplasia protein homolog",
  "gene_symbol": "ACD",
  "term_label": "telomere capping",
  "term_id": "GO:0016233"
}